positive regulation of protein localization to membrane [GO:1905477] (biological process) Subtypes: positive regulation of protein targeting to vacuolar membrane [GO:1900485], positive regulation of protein localization to plasma membrane [GO:1903078], GO:1903569, positive regulation of receptor clustering [GO:1903911], positive regulation of t-SNARE clustering [GO:1904034], positive regulation of protein localization to basolateral plasma membrane [GO:1904510] Relationships: is_a GO:0048522; is a type of positive regulation of protein localization [GO:1903829]; is a type of regulation of protein localization to membrane [GO:1905475]; positively regulates GO:0072657 References: PMID:26911690 Sources: GOC:PARL, GOC:TermGenie, GOC:bc, GO_REF:0000058 Also known as: positive regulation of protein localisation in membrane, positive regulation of protein localization in membrane, up regulation of protein localisation in membrane, up regulation of protein localization in membrane, up regulation of protein localization to membrane, up-regulation of protein localisation in membrane, up-regulation of protein localization in membrane, up-regulation of protein localization to membrane, upregulation of protein localisation in membrane, upregulation of protein localization in membrane, upregulation of protein localization to membrane, activation of protein localisation in membrane, activation of protein localization in membrane, activation of protein localization to membrane Definition: Any process that activates or increases the frequency, rate or extent of protein localization to membrane.